{
  "gene_symbol": "MEF2B",
  "term_label": "cell differentiation",
  "gene_name": "Myocyte-specific enhancer factor 2B",
  "gene": "UniProtKB:Q02080",
  "term_id": "GO:0030154"
}